{
  "term_label": "cytokine activity",
  "term_id": "GO:0005125",
  "gene_name": "Proto-oncogene Wnt-3",
  "gene_symbol": "WNT3",
  "gene": "UniProtKB:P56703"
}